{
  "gene_symbol": "C16orf86",
  "gene_name": "Uncharacterized protein C16orf86",
  "gene": "UniProtKB:Q6ZW13",
  "term_id": "UNKNOWN:0003",
  "term_label": "Unknown cellular component"
}